CD4-positive, alpha-beta T cell cytokine production [GO:0035743] (BP) Note: Note that this term is in the subset of terms that should not be used for direct gene product annotation. Instead, select one of the 'regulation' children terms. Subtypes: GO:0035744, T-helper 2 cell cytokine production [GO:0035745] Definition: Any process that contributes to cytokine production by a CD4-positive, alpha-beta T cell. Sources: CL:0000624, GOC:BHF Relationships: is a type of T cell cytokine production [GO:0002369]